positive regulation of developmental pigmentation [GO:0048087] (biological process) Relationships: is a type of GO:0048070; is a type of positive regulation of biological process [GO:0048518]; positively regulates developmental pigmentation [GO:0048066] Subtypes: positive regulation of eye pigmentation [GO:0048075], positive regulation of cuticle pigmentation [GO:0048081], GO:0048091, positive regulation of male pigmentation [GO:0048093], positive regulation of pigment cell differentiation [GO:0050942] Definition: Any process that increases the frequency, rate or extent of the developmental process that results in the deposition of coloring matter in an organism. Sources: GOC:dph, GOC:jid, GOC:tb Also known as: up regulation of developmental pigmentation, up-regulation of developmental pigmentation, upregulation of developmental pigmentation, activation of developmental pigmentation, stimulation of developmental pigmentation